positive regulation of stress response to copper ion [GO:1903855] (biological process) Also known as: positive regulation of response to copper ion stress, up regulation of response to copper ion stress, up regulation of stress response to copper ion, up-regulation of response to copper ion stress, up-regulation of stress response to copper ion, upregulation of response to copper ion stress, upregulation of stress response to copper ion, activation of response to copper ion stress, activation of stress response to copper ion, activation of response to copper toxicity, positive regulation of response to copper toxicity, up regulation of response to copper toxicity, up-regulation of response to copper toxicity, upregulation of response to copper toxicity Relationships: is a type of positive regulation of response to stimulus [GO:0048584]; is a type of GO:1903853; RO_0002213 stress response to copper ion [GO:1990169] Definition: Any process that activates or increases the frequency, rate or extent of stress response to copper ion. References: PMID:23437011 Sources: GOC:TermGenie, GOC:kmv, GO_REF:0000058